{
  "gene": "UniProtKB:Q14207",
  "term_id": "UNKNOWN:0002",
  "gene_name": "Protein NPAT",
  "gene_symbol": "NPAT",
  "term_label": "Unknown biological process"
}